activation of reciprocal meiotic recombination [GO:0010846] (biological process) Definition: Any process that starts the inactive process of reciprocal meiotic recombination. Reciprocal meiotic recombination is the cell cycle process in which double strand breaks are formed and repaired through a double Holliday junction intermediate. Sources: GOC:dph, GOC:tb Also known as: activation of meiotic recombination Relationships: is a type of positive regulation of reciprocal meiotic recombination [GO:0010845]